response to manganese ion [GO:0010042] (BP) Sources: GOC:sm Subtypes: cellular response to manganese ion [GO:0071287] Relationships: is a type of GO:0010038 Also known as: response to manganese Definition: Any process that results in a change in state or activity of a cell or an organism (in terms of movement, secretion, enzyme production, gene expression, etc.) as a result of a manganese ion stimulus.